{
  "gene": "UniProtKB:P58513",
  "term_label": "Unknown cellular component",
  "term_id": "UNKNOWN:0003",
  "gene_symbol": "LINC00158",
  "gene_name": "Putative uncharacterized protein encoded by LINC00158"
}